{
  "term_label": "receptor clustering",
  "gene_symbol": "AGRN",
  "gene": "UniProtKB:O00468",
  "gene_name": "Agrin",
  "term_id": "GO:0043113"
}